{
  "gene": "UniProtKB:P50549",
  "term_id": "GO:0030154",
  "term_label": "cell differentiation",
  "gene_symbol": "ETV1",
  "gene_name": "ETS translocation variant 1"
}